pollen tube development [GO:0048868] (biological process) Definition: The process whose specific outcome is the progression of a pollen tube over time, from its initial formation to a mature structure. Sources: GOC:isa_complete Relationships: is a type of developmental process involved in reproduction [GO:0003006]; is a type of GO:0048856; BFO_0000050 pollination [GO:0009856]